putrescine biosynthetic process from arginine, via agmatine [GO:0033389] (BP) Sources: GOC:mah, MetaCyc:PWY-40 Relationships: is a type of putrescine biosynthetic process from arginine [GO:0033388] Definition: The chemical reactions and pathways resulting in the formation of putrescine, 1,4-diaminobutane, from arginine via agmatine. Also known as: putrescine anabolism from arginine, using agmatinase, putrescine biosynthesis from arginine, using agmatinase, putrescine biosynthetic process from arginine, using agmatinase, putrescine formation from arginine, using agmatinase, putrescine synthesis from arginine, using agmatinase